{
  "gene_name": "Galectin-8",
  "gene_symbol": "LGALS8",
  "gene": "UniProtKB:O00214",
  "term_id": "UNKNOWN:0002",
  "term_label": "Unknown biological process"
}